positive regulation of smoothened signaling pathway involved in dorsal/ventral neural tube patterning [GO:1901622] (biological process) Also known as: positive regulation of hedgehog signaling pathway involved in dorsal/ventral neural tube patterning, positive regulation of hh signaling pathway involved in dorsal/ventral neural tube patterning, positive regulation of smoothened signalling pathway involved in dorsal/ventral neural tube patterning, up regulation of hedgehog signaling pathway involved in dorsal/ventral neural tube patterning, up regulation of hh signaling pathway involved in dorsal/ventral neural tube patterning, up regulation of smoothened signaling pathway involved in dorsal/ventral neural tube patterning, up regulation of smoothened signalling pathway involved in dorsal/ventral neural tube patterning, up-regulation of hedgehog signaling pathway involved in dorsal/ventral neural tube patterning, up-regulation of hh signaling pathway involved in dorsal/ventral neural tube patterning, up-regulation of smoothened signaling pathway involved in dorsal/ventral neural tube patterning, up-regulation of smoothened signalling pathway involved in dorsal/ventral neural tube patterning, upregulation of hedgehog signaling pathway involved in dorsal/ventral neural tube patterning, upregulation of hh signaling pathway involved in dorsal/ventral neural tube patterning, upregulation of smoothened signaling pathway involved in dorsal/ventral neural tube patterning, upregulation of smoothened signalling pathway involved in dorsal/ventral neural tube patterning, activation of hedgehog signaling pathway involved in dorsal/ventral neural tube patterning, activation of hh signaling pathway involved in dorsal/ventral neural tube patterning, activation of smoothened signaling pathway involved in dorsal/ventral neural tube patterning, activation of smoothened signalling pathway involved in dorsal/ventral neural tube patterning Relationships: is_a positive regulation of smoothened signaling pathway [GO:0045880]; is a type of regulation of smoothened signaling pathway involved in dorsal/ventral neural tube patterning [GO:1901620]; positively regulates smoothened signaling pathway involved in dorsal/ventral neural tube patterning [GO:0060831] Sources: GOC:TermGenie Definition: Any process that activates or increases the frequency, rate or extent of smoothened signaling pathway involved in dorsal/ventral neural tube patterning.